{
  "gene_symbol": "LAMB1",
  "term_id": "GO:0005604",
  "gene": "UniProtKB:P07942",
  "term_label": "basement membrane",
  "gene_name": "Laminin subunit beta-1"
}